demethylsterigmatocystin 6-O-methyltransferase activity [GO:0047145] (molecular function) Relationships: is a type of O-methyltransferase activity [GO:0008171] Sources: EC:2.1.1.109, MetaCyc:2.1.1.109-RXN Also known as: O-methyltransferase I, S-adenosyl-L-methionine:6-demethylsterigmatocystin 6-O-methyltransferase activity, demethylsterigmatocystin methyltransferase activity Definition: Catalysis of the reaction: 6-demethylsterigmatocystin + S-adenosyl-L-methionine = sterigmatocystin + S-adenosyl-homocysteine.